{
  "term_id": "GO:0030424",
  "gene_symbol": "SYT2",
  "term_label": "axon",
  "gene": "UniProtKB:Q8N9I0",
  "gene_name": "Synaptotagmin-2"
}